{
  "gene": "UniProtKB:Q99717",
  "gene_name": "Mothers against decapentaplegic homolog 5",
  "term_label": "I-SMAD binding",
  "term_id": "GO:0070411",
  "gene_symbol": "SMAD5"
}